{
  "gene_name": "Dolichyl-diphosphooligosaccharide--protein glycosyltransferase subunit STT3A",
  "term_label": "protein N-linked glycosylation via asparagine",
  "gene": "UniProtKB:P46977",
  "term_id": "GO:0018279",
  "gene_symbol": "STT3A"
}